amylase secretion [GO:0036394] (biological process) Definition: The controlled release of amylase from a cell. References: PMID:19028687 Sources: GOC:jc Subtypes: pancreatic amylase secretion [GO:0036395] Relationships: is a type of protein secretion [GO:0009306] Also known as: amylase release